{
  "term_label": "positive regulation of transcription by RNA polymerase II",
  "gene_symbol": "GSX1",
  "gene_name": "GS homeobox 1",
  "term_id": "GO:0045944",
  "gene": "UniProtKB:Q9H4S2"
}